{
  "gene_symbol": "NOTO",
  "term_label": "regulation of transcription by RNA polymerase II",
  "term_id": "GO:0006357",
  "gene": "UniProtKB:A8MTQ0",
  "gene_name": "Homeobox protein notochord"
}